{
  "gene_symbol": "PCIF1",
  "gene": "UniProtKB:Q9H4Z3",
  "term_id": "UNKNOWN:0002",
  "term_label": "Unknown biological process",
  "gene_name": "mRNA (2'-O-methyladenosine-N(6)-)-methyltransferase"
}